{
  "term_id": "GO:0001669",
  "gene_symbol": "LY6K",
  "term_label": "acrosomal vesicle",
  "gene_name": "Lymphocyte antigen 6K",
  "gene": "UniProtKB:Q17RY6"
}